{
  "gene_symbol": "NETO2",
  "term_label": "postsynaptic density membrane",
  "term_id": "GO:0098839",
  "gene": "UniProtKB:Q8NC67",
  "gene_name": "Neuropilin and tolloid-like protein 2"
}